{
  "term_label": "replication fork",
  "gene": "UniProtKB:O15315",
  "term_id": "GO:0005657",
  "gene_name": "DNA repair protein RAD51 homolog 2",
  "gene_symbol": "RAD51B"
}